{
  "term_label": "ubiquitin-protein transferase activity",
  "term_id": "GO:0004842",
  "gene_name": "E3 ubiquitin-protein ligase TTC3",
  "gene_symbol": "TTC3",
  "gene": "UniProtKB:P53804"
}